{
  "gene_symbol": "RAC2",
  "term_id": "GO:0007165",
  "gene": "UniProtKB:P15153",
  "term_label": "signal transduction",
  "gene_name": "Ras-related C3 botulinum toxin substrate 2"
}